regulation of starch catabolic process [GO:2000881] (biological process) Also known as: regulation of starch breakdown, regulation of starch catabolism, regulation of starch degradation Subtypes: negative regulation of starch catabolic process [GO:2000882], positive regulation of starch catabolic process [GO:2000883] Definition: Any process that modulates the frequency, rate or extent of starch catabolic process. Relationships: is a type of regulation of carbohydrate catabolic process [GO:0043470]; is a type of GO:2000904; regulates starch catabolic process [GO:0005983] Sources: GOC:obol